{
  "term_label": "sphingosine-1-phosphate phosphatase activity",
  "gene_name": "Inactive phospholipid phosphatase 7",
  "term_id": "GO:0042392",
  "gene": "UniProtKB:Q8NBV4",
  "gene_symbol": "PLPP7"
}